response to L-thialysine [GO:1901345] (biological process) Subtypes: cellular response to L-thialysine [GO:0072751] Sources: GOC:TermGenie Also known as: response to thialysine Definition: Any process that results in a change in state or activity of a cell or an organism (in terms of movement, secretion, enzyme production, gene expression, etc.) as a result of a L-thialysine stimulus. Relationships: is a type of response to amino acid [GO:0043200]; is a type of response to nitrogen compound [GO:1901698]; is a type of GO:1901700